regulation of muscle filament sliding involved in regulation of the velocity of shortening in skeletal muscle contraction [GO:0014880] (biological process) Sources: GOC:dph, GOC:mtg_muscle, GOC:tb Subtypes: cross bridge cycling involved in regulation of the velocity of shortening in skeletal muscle contraction [GO:0014868], GO:0014871, regulation of muscle filament sliding speed involved in regulation of the velocity of shortening in skeletal muscle contraction [GO:0014915] Definition: Any process that modulates the frequency, rate or extent of muscle filament sliding, and consequently contributes to the regulation of the velocity of shortening of skeletal muscle contraction. Relationships: is a type of regulation of muscle filament sliding [GO:0032971]; BFO_0000050 regulation of the velocity of shortening of skeletal muscle modulating contraction [GO:0014729]